{
  "gene": "UniProtKB:A6NJG6",
  "gene_symbol": "ARGFX",
  "term_id": "GO:0000978",
  "gene_name": "Arginine-fifty homeobox",
  "term_label": "RNA polymerase II cis-regulatory region sequence-specific DNA binding"
}